{
  "gene": "UniProtKB:Q9H221",
  "term_id": "GO:0042632",
  "term_label": "cholesterol homeostasis",
  "gene_symbol": "ABCG8",
  "gene_name": "ATP-binding cassette sub-family G member 8"
}